lycopene beta cyclase activity [GO:0045436] (molecular function) Also known as: lycopene cyclase, crtL Definition: Catalysis of the cyclization of beta rings at one or both ends of the lycopene molecule (psi, psi-carotene) to form gamma-carotene or the bicyclic beta-carotene (beta, beta-carotene), respectively. References: PMID:8837512 Relationships: is_a cyclase activity [GO:0009975]; is a type of intramolecular oxidoreductase activity [GO:0016860]